{
  "term_label": "Unknown biological process",
  "gene": "UniProtKB:Q96KF7",
  "gene_symbol": "SMIM8",
  "gene_name": "Small integral membrane protein 8",
  "term_id": "UNKNOWN:0002"
}